{
  "gene": "UniProtKB:Q05084",
  "gene_name": "Islet cell autoantigen 1",
  "gene_symbol": "ICA1",
  "term_id": "GO:0140090",
  "term_label": "membrane curvature sensor activity"
}